organism emergence from protective structure [GO:0071684] (biological process) Relationships: is a type of multicellular organismal process [GO:0032501] Definition: The developmental process in which an organism emerges from a surrounding protective structure such as an egg or pupa case. Sources: GOC:mah Subtypes: GO:0007562, GO:0035188